{
  "gene": "UniProtKB:Q6PII5",
  "term_id": "UNKNOWN:0002",
  "gene_symbol": "HAGHL",
  "gene_name": "Hydroxyacylglutathione hydrolase-like protein",
  "term_label": "Unknown biological process"
}